{
  "term_label": "Unknown biological process",
  "term_id": "UNKNOWN:0002",
  "gene_symbol": "REX1BD",
  "gene_name": "Required for excision 1-B domain-containing protein",
  "gene": "UniProtKB:Q96EN9"
}